{
  "gene": "UniProtKB:Q86XA9",
  "gene_symbol": "HEATR5A",
  "gene_name": "HEAT repeat-containing protein 5A",
  "term_label": "endocytic vesicle",
  "term_id": "GO:0030139"
}